{
  "gene": "UniProtKB:O43711",
  "gene_symbol": "TLX3",
  "term_id": "GO:0048513",
  "term_label": "animal organ development",
  "gene_name": "T-cell leukemia homeobox protein 3"
}